{
  "gene": "UniProtKB:Q92963",
  "gene_name": "GTP-binding protein Rit1",
  "term_id": "GO:0007265",
  "gene_symbol": "RIT1",
  "term_label": "Ras protein signal transduction"
}